{
  "gene_symbol": "RENBP",
  "term_id": "UNKNOWN:0002",
  "gene_name": "N-acylglucosamine 2-epimerase",
  "gene": "UniProtKB:P51606",
  "term_label": "Unknown biological process"
}